{
  "gene_name": "Double zinc ribbon and ankyrin repeat-containing protein 1",
  "gene_symbol": "DZANK1",
  "term_label": "Unknown molecular function",
  "term_id": "UNKNOWN:0001",
  "gene": "UniProtKB:Q9NVP4"
}